{
  "term_label": "cytoplasm",
  "gene_name": "Phospholipase A-2-activating protein",
  "gene_symbol": "PLAA",
  "term_id": "GO:0005737",
  "gene": "UniProtKB:Q9Y263"
}